{
  "gene_name": "Transmembrane protein 203",
  "term_id": "UNKNOWN:0001",
  "gene": "UniProtKB:Q969S6",
  "term_label": "Unknown molecular function",
  "gene_symbol": "TMEM203"
}